{
  "gene_symbol": "ARMH1",
  "term_id": "UNKNOWN:0002",
  "gene": "UniProtKB:Q6PIY5",
  "gene_name": "Armadillo-like helical domain containing protein 1",
  "term_label": "Unknown biological process"
}